{
  "gene_name": "Ras-related GTP-binding protein C",
  "gene_symbol": "RRAGC",
  "term_label": "cellular response to starvation",
  "gene": "UniProtKB:Q9HB90",
  "term_id": "GO:0009267"
}